{
  "gene_name": "Bifunctional 3'-phosphoadenosine 5'-phosphosulfate synthase 1",
  "gene": "UniProtKB:O43252",
  "term_label": "3'-phosphoadenosine 5'-phosphosulfate biosynthetic process",
  "term_id": "GO:0050428",
  "gene_symbol": "PAPSS1"
}